{
  "term_label": "Unknown biological process",
  "gene_name": "T cell receptor alpha joining 28 (Fragment)",
  "gene": "UniProtKB:A0A075B6X4",
  "term_id": "UNKNOWN:0002",
  "gene_symbol": "TRAJ28"
}